magnesium-protoporphyrin IX monomethyl ester (oxidative) cyclase activity [GO:0048529] (molecular function) Definition: Catalysis of the reaction: magnesium protoporphyrin IX 13-monomethyl ester + 3 NADPH + 3 H+ + 3 O2 = divinylprotochlorophyllide + 3 NADP+ + 5 H2O. Sources: EC:1.14.13.81, RHEA:33235 Relationships: is a type of GO:0016709 Also known as: Mg-protoporphyrin IX monomethyl ester (oxidative) cyclase activity, Mg-protoporphyrin IX monomethyl ester oxidative cyclase activity, magnesium-protoporphyrin-IX 13-monomethyl ester,NADPH:oxygen oxidoreductase (hydroxylating)